regulation of DNA biosynthetic process [GO:2000278] (biological process) Relationships: is_a regulation of macromolecule biosynthetic process [GO:0010556]; is a type of regulation of DNA metabolic process [GO:0051052]; regulates DNA biosynthetic process [GO:0071897] Also known as: regulation of DNA anabolism, regulation of DNA biosynthesis, regulation of DNA formation, regulation of DNA synthesis Definition: Any process that modulates the frequency, rate or extent of DNA biosynthetic process. Subtypes: GO:0032210, regulation of reverse transcription [GO:1900268], regulation of error-prone translesion synthesis [GO:1904331], regulation of DNA amplification [GO:1904523], GO:2000279, positive regulation of DNA biosynthetic process [GO:2000573] Sources: GOC:obol